Ac-Asp-Glu binding [GO:1904492] (molecular function) Definition: Binding to Ac-Asp-Glu. References: PMID:24863754 Sources: GOC:BHF, GOC:TermGenie, GOC:hal, GO_REF:0000067 Relationships: is a type of anion binding [GO:0043168]; is a type of oligopeptide binding [GO:1900750]